negative regulation of protein binding [GO:0032091] (biological process) Subtypes: GO:1900121, GO:1904530 Definition: Any process that stops, prevents, or reduces the frequency, rate or extent of protein binding. Sources: GOC:mah Relationships: is_a regulation of protein binding [GO:0043393]; is a type of negative regulation of binding [GO:0051100]; negatively regulates protein binding [GO:0005515] Also known as: down regulation of protein binding, down-regulation of protein binding, downregulation of protein binding, inhibition of protein binding